{
  "term_label": "regulation of JNK cascade",
  "term_id": "GO:0046328",
  "gene_symbol": "MDFIC2",
  "gene": "UniProtKB:A0A1B0GVS7",
  "gene_name": "MyoD family inhibitor domain-containing protein 2"
}